polymannuronate hydrolase activity [GO:0033936] (molecular function) Also known as: poly(mannuronide) mannuronohydrolase activity, polymannuronic acid polymerase activity Definition: Catalysis of the endohydrolysis of the D-mannuronide linkages of polymannuronate. Sources: EC:3.2.1.121 Relationships: is a type of GO:0004553